{
  "gene_name": "P2X purinoceptor 7",
  "term_label": "extracellularly ATP-gated monoatomic cation channel activity",
  "gene_symbol": "P2RX7",
  "term_id": "GO:0004931",
  "gene": "UniProtKB:Q99572"
}